response to irinotecan [GO:0061482] (biological process) Relationships: is a type of GO:0042221 Definition: Any process that results in a change in state or activity of a cell or an organism (in terms of movement, secretion, enzyme production, gene expression, etc.) as a result of an irinotecan stimulus. Sources: GOC:dph